polyamine oxidase activity [GO:0046592] (molecular function) Relationships: is a type of GO:0016647 Subtypes: N8-acetylspermidine:oxygen oxidoreductase (propane-1,3-diamine-forming) activity [GO:0052897], spermine oxidase (propane-1,3-diamine-forming) activity [GO:0052900], GO:0052901, N(1)-acetylpolyamine oxidase (3-acetamidopropanal-forming) activity [GO:0052903], thermospermine oxidase activity [GO:1990534] References: PMID:1567380 Definition: Catalysis of the oxidative degradation or interconversion of polyamines. Also known as: 1-N-acetylspermidine:oxygen oxidoreductase (deaminating), N1-acetylspermidine:oxygen oxidoreductase (deaminating)